ATP-binding cassette (ABC) transporter complex, transmembrane substrate-binding subunit-containing [GO:0035796] (cellular component) Relationships: is a type of ATP-binding cassette (ABC) transporter complex [GO:0043190] References: PMID:18931129, PMID:20972419, PMID:21135102 Also known as: ATP-binding cassette (ABC) transporter complex, ECF-type, energy coupling factor (ECF)-type ABC transporter, energy-coupling factor transporter Note: The ECF-type transporters differs from other types of ABC transporters because the substrate-binding subunit lies integral to the membrane. Definition: A complex for the transport of metabolites into the cell, consisting of 4 subunits: a transmembrane substrate-binding protein (known as the S component), and an energy-coupling module that comprises two ATP-binding proteins (known as the A and A' components) and a transmembrane protein (known as the T component). Transport of the substrate across the membrane is driven by the hydrolysis of ATP.